{
  "gene": "UniProtKB:Q96EV8",
  "term_label": "anterograde synaptic vesicle transport",
  "gene_name": "Dysbindin",
  "gene_symbol": "DTNBP1",
  "term_id": "GO:0048490"
}